{
  "gene_symbol": "HAP1",
  "gene_name": "Huntingtin-associated protein 1",
  "term_label": "mitochondrion",
  "gene": "UniProtKB:P54257",
  "term_id": "GO:0005739"
}